{
  "term_label": "water transport",
  "gene_symbol": "AQP8",
  "term_id": "GO:0006833",
  "gene": "UniProtKB:O94778",
  "gene_name": "Aquaporin-8"
}